{
  "gene": "UniProtKB:Q86V88",
  "gene_symbol": "MDP1",
  "term_id": "UNKNOWN:0002",
  "term_label": "Unknown biological process",
  "gene_name": "Magnesium-dependent phosphatase 1"
}